spike train [GO:0098874] (biological process) Relationships: is a type of regulation of membrane potential [GO:0042391]; has part action potential [GO:0001508] Definition: A series of sequential, propagated action potentials occurring in a single cell. Regulation: regulated by regulation of action potential firing pattern [GO:0099608] Sources: ISBN:978-0071390118 Also known as: burst of action potentials, spike-train